{
  "term_id": "GO:0141162",
  "gene": "UniProtKB:P27815",
  "gene_symbol": "PDE4A",
  "gene_name": "cAMP-specific 3',5'-cyclic phosphodiesterase 4A",
  "term_label": "negative regulation of cAMP/PKA signal transduction"
}